visually-mediated background adaptation [GO:0120303] (biological process) Definition: Any process in which an organism changes its pigmentation (lightening in response to a brighter environment or darkening in response to a dimmer environment) in response to a change in light intensity detected by melanopsin-expressing eye cells. Relationships: is a type of background adaptation [GO:0120302] References: PMID:29239123, PMID:32898924 Sources: GOC:cvs, GOC:krc